{
  "gene_symbol": "NABP1",
  "term_label": "mitotic G2/M transition checkpoint",
  "term_id": "GO:0044818",
  "gene_name": "SOSS complex subunit B2",
  "gene": "UniProtKB:Q96AH0"
}